cellular response to misfolded protein [GO:0071218] (biological process) Sources: GOC:mah Definition: Any process that results in a change in state or activity of a cell (in terms of movement, secretion, enzyme production, gene expression, etc.) as a result of a misfolded protein stimulus. Relationships: is_a cellular response to topologically incorrect protein [GO:0035967]; is a type of response to misfolded protein [GO:0051788]